{
  "term_id": "GO:0043235",
  "gene_symbol": "GPRC5B",
  "gene": "UniProtKB:Q9NZH0",
  "gene_name": "G-protein coupled receptor family C group 5 member B",
  "term_label": "receptor complex"
}